{
  "term_id": "GO:0006357",
  "gene_symbol": "SIX6",
  "gene": "UniProtKB:O95475",
  "term_label": "regulation of transcription by RNA polymerase II",
  "gene_name": "Homeobox protein SIX6"
}